{
  "term_id": "GO:0016477",
  "term_label": "cell migration",
  "gene_name": "Crk-like protein",
  "gene_symbol": "CRKL",
  "gene": "UniProtKB:P46109"
}